left nucleus [GO:0097571] (cellular component) Note: Due to the asymmetric nature of the Giardia trophozoite, this term is defined spatially as the trophozoite is viewed from the dorsal side, with the two nuclei dorsal to the ventral disc, and the ventral disc toward the anterior. Sources: GOC:giardia, ISBN:0-444-81258-X Definition: One of the two nuclei found in Giardia species (trophozoite stage). It is located on the left side of the cell when viewed from the dorsal side. Relationships: is a type of GO:0005634